{
  "gene": "UniProtKB:Q2TAP0",
  "gene_symbol": "GOLGA7B",
  "term_id": "GO:0002178",
  "term_label": "palmitoyltransferase complex",
  "gene_name": "Golgin subfamily A member 7B"
}